{
  "term_id": "GO:0003724",
  "term_label": "RNA helicase activity",
  "gene_name": "U5 small nuclear ribonucleoprotein 200 kDa helicase",
  "gene_symbol": "SNRNP200",
  "gene": "UniProtKB:O75643"
}